{
  "gene_symbol": "PTPN20",
  "term_id": "UNKNOWN:0001",
  "gene_name": "Tyrosine-protein phosphatase non-receptor type 20",
  "term_label": "Unknown molecular function",
  "gene": "UniProtKB:Q4JDL3"
}